{
  "gene": "UniProtKB:Q7L273",
  "gene_symbol": "KCTD9",
  "term_id": "UNKNOWN:0001",
  "term_label": "Unknown molecular function",
  "gene_name": "BTB_POZ domain-containing protein KCTD9"
}